microtubule polymerization based protein transport [GO:0099112] (biological process) Relationships: is_a intracellular protein transport [GO:0006886]; is a type of microtubule-based process [GO:0007017]; is a type of microtubule-based protein transport [GO:0099118]; has part GO:0046785 Definition: The transport of a protein driven by polymerization of a microtubule to which it is attached. Subtypes: microtubule polymerization based protein transport to cell tip cortex [GO:0099110] References: PMID:11018050 Sources: GOC:dos, GOC:vw